{
  "term_id": "GO:0005886",
  "gene_symbol": "CCKAR",
  "term_label": "plasma membrane",
  "gene_name": "Cholecystokinin receptor type A",
  "gene": "UniProtKB:P32238"
}